{
  "term_id": "GO:0005789",
  "gene_symbol": "TMEM38B",
  "gene": "UniProtKB:Q9NVV0",
  "gene_name": "Trimeric intracellular cation channel type B",
  "term_label": "endoplasmic reticulum membrane"
}